{
  "gene_symbol": "S100A12",
  "gene": "UniProtKB:P80511",
  "term_id": "GO:0043542",
  "gene_name": "Protein S100-A12",
  "term_label": "endothelial cell migration"
}